{
  "term_id": "UNKNOWN:0001",
  "gene": "UniProtKB:Q969X6",
  "gene_name": "U3 small nucleolar RNA-associated protein 4 homolog",
  "gene_symbol": "UTP4",
  "term_label": "Unknown molecular function"
}